{
  "term_id": "GO:0060828",
  "gene_symbol": "CCNY",
  "gene": "UniProtKB:Q8ND76",
  "term_label": "regulation of canonical Wnt signaling pathway",
  "gene_name": "Cyclin-Y"
}